{
  "term_id": "UNKNOWN:0001",
  "gene_symbol": "VPS37A",
  "gene_name": "Vacuolar protein sorting-associated protein 37A",
  "term_label": "Unknown molecular function",
  "gene": "UniProtKB:Q8NEZ2"
}